{
  "term_id": "GO:0019731",
  "gene_symbol": "SLPI",
  "term_label": "antibacterial humoral response",
  "gene_name": "Antileukoproteinase",
  "gene": "UniProtKB:P03973"
}